{
  "gene_symbol": "ENC1",
  "gene": "UniProtKB:O14682",
  "gene_name": "Ectoderm-neural cortex protein 1",
  "term_id": "GO:0010499",
  "term_label": "proteasomal ubiquitin-independent protein catabolic process"
}